{
  "gene_symbol": "HEATR6",
  "term_id": "UNKNOWN:0002",
  "gene": "UniProtKB:Q6AI08",
  "gene_name": "HEAT repeat-containing protein 6",
  "term_label": "Unknown biological process"
}